positive regulation of Toll receptor ligand protein activation cascade [GO:0160034] (biological process) Relationships: is a type of regulation of Toll receptor ligand protein activation cascade [GO:0160033]; is a type of positive regulation of protein activation cascade [GO:2000259]; positively regulates Toll receptor ligand protein activation cascade [GO:0160032] Definition: Any process that activates or increases the frequency, rate or extent of Toll receptor ligand protein activation cascade. References: PMID:23632253